{
  "term_id": "GO:0006749",
  "gene_symbol": "GSTA3",
  "gene_name": "Glutathione S-transferase A3",
  "term_label": "glutathione metabolic process",
  "gene": "UniProtKB:Q16772"
}